{
  "gene": "UniProtKB:O95777",
  "gene_symbol": "LSM8",
  "gene_name": "U6 snRNA-associated Sm-like protein LSm8",
  "term_id": "GO:0005688",
  "term_label": "U6 snRNP"
}